{
  "term_id": "UNKNOWN:0001",
  "gene_name": "Density-regulated protein",
  "gene": "UniProtKB:O43583",
  "gene_symbol": "DENR",
  "term_label": "Unknown molecular function"
}